{
  "gene_symbol": "PRMT2",
  "gene": "UniProtKB:P55345",
  "term_label": "protein-arginine N-methyltransferase activity",
  "term_id": "GO:0016274",
  "gene_name": "Protein arginine N-methyltransferase 2"
}